{
  "gene": "UniProtKB:P50914",
  "term_id": "GO:0042273",
  "gene_name": "Large ribosomal subunit protein eL14",
  "gene_symbol": "RPL14",
  "term_label": "ribosomal large subunit biogenesis"
}